{
  "gene": "UniProtKB:Q8N3L3",
  "gene_name": "Beta-taxilin",
  "gene_symbol": "TXLNB",
  "term_id": "UNKNOWN:0003",
  "term_label": "Unknown cellular component"
}